G protein-coupled dopamine receptor signaling pathway [GO:0007212] (biological process) Relationships: is a type of G protein-coupled receptor signaling pathway [GO:0007186]; is part of cellular response to dopamine [GO:1903351]; has part synaptic transmission, dopaminergic [GO:0001963] Regulation: regulated by regulation of dopamine receptor signaling pathway [GO:0060159]; negatively regulated by negative regulation of dopamine receptor signaling pathway [GO:0060160]; positively regulated by positive regulation of dopamine receptor signaling pathway [GO:0060161] References: PMID:36757901 Also known as: dopamine receptor signalling pathway Subtypes: adenylate cyclase-activating dopamine receptor signaling pathway [GO:0007191], GO:0007195, phospholipase C-activating dopamine receptor signaling pathway [GO:0060158] Definition: A G protein-coupled receptor signaling pathway initiated by a dopamine binding to its receptor on the surface of a target cell, and ending with the regulation of a downstream cellular process.